tRNA end turnover [GO:0042778] (BP) Relationships: is a type of GO:0006399 Definition: The process in which the 3'-terminal CCA of a tRNA is removed and restored. This often happens to uncharged tRNA. Sources: GOC:go_curators